{
  "gene_symbol": "AZIN2",
  "gene": "UniProtKB:Q96A70",
  "term_label": "negative regulation of protein catabolic process",
  "term_id": "GO:0042177",
  "gene_name": "Antizyme inhibitor 2"
}